{
  "gene_name": "GATOR complex protein WDR59",
  "gene": "UniProtKB:Q6PJI9",
  "term_label": "positive regulation of TORC1 signaling",
  "term_id": "GO:1904263",
  "gene_symbol": "WDR59"
}